{
  "gene_symbol": "COA3",
  "gene_name": "Cytochrome c oxidase assembly factor 3 homolog, mitochondrial",
  "term_id": "UNKNOWN:0001",
  "gene": "UniProtKB:Q9Y2R0",
  "term_label": "Unknown molecular function"
}